{
  "term_label": "enzyme inhibitor activity",
  "term_id": "GO:0004857",
  "gene_name": "UDP-glucuronosyltransferase 1A5",
  "gene_symbol": "UGT1A5",
  "gene": "UniProtKB:P35504"
}